{
  "term_label": "nucleus",
  "term_id": "GO:0005634",
  "gene_symbol": "ZIM3",
  "gene_name": "Zinc finger imprinted 3",
  "gene": "UniProtKB:Q96PE6"
}